{
  "gene_symbol": "MTMR9",
  "gene": "UniProtKB:Q96QG7",
  "gene_name": "Myotubularin-related protein 9",
  "term_id": "GO:0010507",
  "term_label": "negative regulation of autophagy"
}